{
  "term_label": "peptidoglycan immune receptor activity",
  "gene": "UniProtKB:Q96LB9",
  "gene_name": "Peptidoglycan recognition protein 3",
  "gene_symbol": "PGLYRP3",
  "term_id": "GO:0016019"
}